{
  "gene_symbol": "LENEP",
  "gene": "UniProtKB:Q9Y5L5",
  "term_id": "UNKNOWN:0001",
  "term_label": "Unknown molecular function",
  "gene_name": "Lens epithelial cell protein LEP503"
}